{
  "gene": "UniProtKB:Q9C004",
  "term_label": "protein kinase inhibitor activity",
  "gene_symbol": "SPRY4",
  "term_id": "GO:0004860",
  "gene_name": "Protein sprouty homolog 4"
}